{
  "term_id": "GO:0005730",
  "gene": "UniProtKB:Q9H6R0",
  "term_label": "nucleolus",
  "gene_symbol": "DHX33",
  "gene_name": "ATP-dependent RNA helicase DHX33"
}